{
  "gene_name": "RuvB-like 1",
  "term_id": "GO:0006357",
  "gene": "UniProtKB:Q9Y265",
  "term_label": "regulation of transcription by RNA polymerase II",
  "gene_symbol": "RUVBL1"
}